regulation of hair follicle cell proliferation [GO:0071336] (biological process) Definition: Any process that modulates the frequency, rate or extent of hair follicle cell proliferation. Sources: GOC:mah Subtypes: negative regulation of hair follicle cell proliferation [GO:0071337], positive regulation of hair follicle cell proliferation [GO:0071338] Relationships: is a type of regulation of cell population proliferation [GO:0042127]; RO_0002211 hair follicle cell proliferation [GO:0071335]